bis(5'-nucleosyl)-tetraphosphatase (asymmetrical) activity [GO:0004081] (MF) Also known as: Ap(4)A hydrolase activity, Ap(4)Aase activity, Ap4A hydrolase activity, Ap4Aase activity, bis(5'-adenosyl)-tetraphosphatase activity, bis(5'-guanosyl)-tetraphosphatase activity, diadenosine 5',5'''-P1,P4-tetraphosphate hydrolase, diadenosinetetraphosphatase (asymmetrical) activity, diguanosinetetraphosphatase (asymmetrical) activity, 1-P,4-P-bis(5'-nucleosyl)-tetraphosphate nucleotidohydrolase activity, P1,P4-bis(5'-nucleosyl)-tetraphosphate nucleotidohydrolase activity, diadenosine 5',5'''-P(1),P(4)-tetraphosphate asymmetrical hydrolase activity, diadenosine 5',5'''-P1,P4-tetraphosphate asymmetrical hydrolase activity, diadenosine P1,P4-tetraphosphatase activity, dinucleoside tetraphosphatase activity, dinucleosidetetraphosphatase (asymmetrical) activity References: PMID:4955726 Sources: EC:3.6.1.17 Relationships: is a type of bis(5'-nucleosyl)-tetraphosphatase activity [GO:0008796] Definition: Catalysis of the reaction: P(1),P(4)-bis(5'-nucleosyl)tetraphosphate + H2O = NTP + NMP. Acts on bis(5'-guanosyl)-, bis(5'-xanthosyl)-, bis(5'-adenosyl)- and bis(5'-uridyl)-tetraphosphate.